{
  "gene_name": "Zinc finger and SCAN domain-containing protein 9",
  "gene_symbol": "ZSCAN9",
  "gene": "UniProtKB:O15535",
  "term_label": "Unknown cellular component",
  "term_id": "UNKNOWN:0003"
}